{
  "gene_name": "Zinc finger transcription factor Trps1",
  "gene": "UniProtKB:Q9UHF7",
  "term_label": "regulation of transcription by RNA polymerase II",
  "term_id": "GO:0006357",
  "gene_symbol": "TRPS1"
}